positive regulation of type 2 immune response [GO:0002830] (biological process) Definition: Any process that activates or increases the frequency, rate, or extent of a type 2 immune response. Sources: GOC:add Also known as: up regulation of type 2 immune response, up-regulation of type 2 immune response, upregulation of type 2 immune response, activation of type 2 immune response, positive regulation of T-helper 2 type immune response, positive regulation of Th2 immune response, stimulation of type 2 immune response Relationships: is a type of regulation of type 2 immune response [GO:0002828]; is a type of positive regulation of immune response [GO:0050778]; positively regulates type 2 immune response [GO:0042092] Subtypes: positive regulation of T-helper 2 cell differentiation [GO:0045630], GO:2000553